{
  "term_id": "GO:0043495",
  "gene": "UniProtKB:Q96BY7",
  "term_label": "protein-membrane adaptor activity",
  "gene_symbol": "ATG2B",
  "gene_name": "Autophagy-related protein 2 homolog B"
}